{
  "gene": "UniProtKB:O95445",
  "gene_name": "Apolipoprotein M",
  "term_id": "GO:0034375",
  "gene_symbol": "APOM",
  "term_label": "high-density lipoprotein particle remodeling"
}